negative regulation of nitrosative stress-induced intrinsic apoptotic signaling pathway [GO:1905259] (biological process) References: PMID:14752510 Sources: GOC:PARL, GOC:TermGenie, GOC:bf, GO_REF:0000058 Definition: Any process that stops, prevents or reduces the frequency, rate or extent of intrinsic apoptotic signaling pathway in response to nitrosative stress. Also known as: down regulation of intrinsic apoptotic signaling pathway in response to nitrosative stress, down regulation of nitrosative stress-induced intrinsic apoptotic signaling pathway, down-regulation of intrinsic apoptotic signaling pathway in response to nitrosative stress, down-regulation of nitrosative stress-induced intrinsic apoptotic signaling pathway, downregulation of intrinsic apoptotic signaling pathway in response to nitrosative stress, downregulation of nitrosative stress-induced intrinsic apoptotic signaling pathway, negative regulation of intrinsic apoptotic signaling pathway in response to nitrosative stress, inhibition of intrinsic apoptotic signaling pathway in response to nitrosative stress, inhibition of nitrosative stress-induced intrinsic apoptotic signaling pathway, down regulation of nitrosative stress-induced apoptosis, down-regulation of nitrosative stress-induced apoptosis, downregulation of nitrosative stress-induced apoptosis, inhibition of nitrosative stress-induced apoptosis, negative regulation of nitrosative stress-induced apoptosis Relationships: is a type of regulation of nitrosative stress-induced intrinsic apoptotic signaling pathway [GO:1905258]; is a type of GO:2001243; negatively regulates intrinsic apoptotic signaling pathway in response to nitrosative stress [GO:1990442]